positive regulation of response to benzene [GO:1901453] (biological process) Relationships: is a type of positive regulation of response to stimulus [GO:0048584]; is a type of regulation of response to benzene [GO:1901451]; positively regulates GO:1901423 Sources: GOC:TermGenie, GOC:mengo_curators Definition: Any process that activates or increases the frequency, rate or extent of response to benzene. Also known as: up regulation of response to benzene, up-regulation of response to benzene, upregulation of response to benzene, activation of response to benzene